{
  "gene_symbol": "BCDIN3D",
  "gene": "UniProtKB:Q7Z5W3",
  "term_id": "GO:0005737",
  "gene_name": "RNA 5'-monophosphate methyltransferase",
  "term_label": "cytoplasm"
}